zinc ion import into mitochondrion [GO:0140917] (biological process) Relationships: is a type of GO:0062111 Definition: The directed import of zinc(2+) from the cytosol, across an organelle membrane, into a mitochondrion. References: PMID:21289295